{
  "gene": "UniProtKB:Q8NGZ9",
  "term_id": "GO:0004984",
  "gene_symbol": "OR2T10",
  "term_label": "olfactory receptor activity",
  "gene_name": "Olfactory receptor 2T10"
}